cellular component maintenance [GO:0043954] (biological process) Relationships: is a type of GO:0016043 Sources: GOC:dph, GOC:jl, GOC:mah Subtypes: actomyosin contractile ring maturation [GO:0031566], cell junction maintenance [GO:0034331], GO:0062195, endoplasmic reticulum cisternal network maintenance [GO:0071785], endoplasmic reticulum tubular network maintenance [GO:0071788], dendritic spine maintenance [GO:0097062], stereocilium maintenance [GO:0120045] Definition: The organization process that preserves a cellular component in a stable functional or structural state. Also known as: cellular component maintenance at cellular level